{
  "term_label": "Unknown biological process",
  "gene_name": "Olfactory receptor 14A16",
  "gene_symbol": "OR14A16",
  "term_id": "UNKNOWN:0002",
  "gene": "UniProtKB:Q8NHC5"
}